{
  "term_id": "GO:0071222",
  "gene": "UniProtKB:Q8NFZ5",
  "gene_symbol": "TNIP2",
  "gene_name": "TNFAIP3-interacting protein 2",
  "term_label": "cellular response to lipopolysaccharide"
}